{
  "term_label": "phosphatidylinositol-3-phosphate phosphatase activity",
  "gene_symbol": "MTM1",
  "gene": "UniProtKB:Q13496",
  "gene_name": "Myotubularin",
  "term_id": "GO:0004438"
}